{
  "gene_symbol": "APEX2",
  "gene": "UniProtKB:Q9UBZ4",
  "term_label": "base-excision repair",
  "term_id": "GO:0006284",
  "gene_name": "DNA-(apurinic or apyrimidinic site) endonuclease 2"
}